heart induction [GO:0003129] (biological process) Sources: GOC:mtg_heart Definition: The close range interaction between mesoderm and endoderm or ectoderm that causes cells to change their fates and specify the development of the heart. Relationships: is a type of GO:0001759; is a type of regulation of heart morphogenesis [GO:2000826]; positively regulates GO:0003128 Regulation: regulated by regulation of heart induction [GO:0090381]; negatively regulated by negative regulation of heart induction [GO:1901320]; positively regulated by GO:1901321